{
  "term_label": "extracellular space",
  "term_id": "GO:0005615",
  "gene": "UniProtKB:O43323",
  "gene_name": "Desert hedgehog protein",
  "gene_symbol": "DHH"
}